calmodulin-activated 3',5'-cyclic-AMP phosphodiesterase activity [GO:0140761] (molecular function) Also known as: calcium- and calmodulin-regulated 3',5'-cyclic-AMP phosphodiesterase activity, calcium- and calmodulin-regulated AMP-specific phosphodiesterase activity, calcium- and calmodulin-regulated cyclic-AMP phosphodiesterase activity, calcium/calmodulin-regulated cAMP-specific phosphodiesterase activity, calcium- and calmodulin-regulated cAMP phosphodiesterase activity Relationships: is_a 3',5'-cyclic-AMP phosphodiesterase activity [GO:0004115] Definition: Catalysis of the reactions: nucleoside 3',5'-cyclic AMP + H2O = AMP + H+; this activity is activated by binding to calcium-bound calmodulin. References: PMID:15901640